sequestering of BMP in extracellular matrix [GO:0035582] (biological process) Note: Confining BMP in the extracellular matrix may be achieved by binding BMP directly, or by binding to members of a BMP-containing complex. Definition: Confining a bone morphogenetic protein (BMP) to the extracellular matrix (ECM), such that it is separated from other components of the signaling pathway, including its cell surface receptor. Bone morphogenetic proteins (BMPs) are secreted as homodimers, non-covalently associated with N-terminal pro-peptides, and are targeted to the extracellular matrix through interaction with matrix proteins. Also known as: BMP sequestration in the ECM, negative regulation of BMP signaling pathway by extracellular sequestering of BMP, negative regulation of BMP signalling pathway by extracellular matrix sequestering of BMP, negative regulation of bone morphogenetic protein signaling pathway by extracellular matrix sequestering of bone morphogenetic protein References: PMID:20855508 Sources: GOC:BHF Relationships: is a type of negative regulation of BMP signaling pathway [GO:0030514]; is a type of sequestering of extracellular ligand from receptor [GO:0035581]; is_a GO:0071694